phosphatidylglycerol transfer activity [GO:0140339] (molecular function) Relationships: is a type of phospholipid transfer activity [GO:0120014] Also known as: phosphatidylglycerol carrier activity Definition: Directly binding to phosphatidylglycerol and delivering it either to an acceptor molecule or to a specific location. References: PMID:9132017